purine nucleoside monophosphate catabolic process [GO:0009128] (biological process) Subtypes: purine ribonucleoside monophosphate catabolic process [GO:0009169], purine deoxyribonucleoside monophosphate catabolic process [GO:0009172] Relationships: is a type of GO:0009125; is a type of purine nucleoside monophosphate metabolic process [GO:0009126] Definition: The chemical reactions and pathways resulting in the breakdown of purine nucleoside monophosphate, a compound consisting of a purine base linked to a ribose or deoxyribose sugar esterified with phosphate on the sugar. Sources: GOC:go_curators, ISBN:0198506732 Also known as: purine nucleoside monophosphate breakdown, purine nucleoside monophosphate catabolism, purine nucleoside monophosphate degradation